{
  "term_id": "GO:0007040",
  "gene_name": "Transcription factor EB",
  "gene_symbol": "TFEB",
  "gene": "UniProtKB:P19484",
  "term_label": "lysosome organization"
}